{
  "term_label": "Unknown molecular function",
  "term_id": "UNKNOWN:0001",
  "gene_symbol": "SNX32",
  "gene": "UniProtKB:Q86XE0",
  "gene_name": "Sorting nexin-32"
}